{
  "gene": "UniProtKB:Q8TAB3",
  "gene_name": "Protocadherin-19",
  "term_id": "GO:0007155",
  "term_label": "cell adhesion",
  "gene_symbol": "PCDH19"
}